{
  "gene_name": "Inward rectifier potassium channel 16",
  "term_id": "UNKNOWN:0001",
  "gene_symbol": "KCNJ16",
  "gene": "UniProtKB:Q9NPI9",
  "term_label": "Unknown molecular function"
}